{
  "gene_name": "BLOC-2 complex member HPS6",
  "gene_symbol": "HPS6",
  "gene": "UniProtKB:Q86YV9",
  "term_label": "lysosome localization",
  "term_id": "GO:0032418"
}